{
  "term_label": "energy homeostasis",
  "term_id": "GO:0097009",
  "gene_name": "Peroxisome proliferator-activated receptor gamma coactivator 1-beta",
  "gene_symbol": "PPARGC1B",
  "gene": "UniProtKB:Q86YN6"
}